{
  "gene_symbol": "ZAN",
  "term_label": "extracellular matrix",
  "gene_name": "Zonadhesin",
  "term_id": "GO:0031012",
  "gene": "UniProtKB:Q9Y493"
}